{
  "gene": "UniProtKB:O76021",
  "gene_symbol": "RSL1D1",
  "gene_name": "Ribosomal L1 domain-containing protein 1",
  "term_id": "GO:0005730",
  "term_label": "nucleolus"
}